{
  "gene": "UniProtKB:Q9HBG4",
  "term_id": "GO:0007035",
  "term_label": "vacuolar acidification",
  "gene_symbol": "ATP6V0A4",
  "gene_name": "V-type proton ATPase 116 kDa subunit a 4"
}